{
  "term_id": "GO:0007097",
  "gene": "UniProtKB:Q9UKB1",
  "gene_symbol": "FBXW11",
  "term_label": "nuclear migration",
  "gene_name": "F-box_WD repeat-containing protein 11"
}